epididymis development [GO:1905867] (BP) References: PMID:12388089 Sources: GOC:TermGenie, GO_REF:0000094 Relationships: is a type of tube development [GO:0035295] Also known as: epididymus development Definition: The process whose specific outcome is the progression of an epididymis over time, from its formation to the mature structure.